{
  "gene_symbol": "RNASE1",
  "gene_name": "Ribonuclease pancreatic",
  "term_id": "GO:0004540",
  "term_label": "RNA nuclease activity",
  "gene": "UniProtKB:P07998"
}